{
  "gene": "UniProtKB:P52895",
  "gene_name": "Aldo-keto reductase family 1 member C2",
  "term_label": "ketosteroid monooxygenase activity",
  "gene_symbol": "AKR1C2",
  "term_id": "GO:0047086"
}